skeletal muscle thin filament assembly [GO:0030240] (biological process) Definition: The aggregation, arrangement and bonding together of proteins to form the actin-based thin filaments of myofibrils in skeletal muscle. Sources: GOC:ef, GOC:mah, GOC:mtg_muscle Relationships: is a type of actin filament organization [GO:0007015]; is part of skeletal myofibril assembly [GO:0014866]